SA node cell to atrial cardiac muscle cell communication [GO:0086070] (biological process) Relationships: is a type of GO:0086065 Sources: GOC:BHF, GOC:mtg_cardiac_conduct_nov11 Subtypes: GO:0086018, SA node cell to atrial cardiac muscle cell communication by electrical coupling [GO:0086021] Definition: The process that mediates interactions between an SA node cardiomyocyte and its surroundings that contributes to the process of the SA node cardiomyocyte communicating with an atrial cardiomyocyte in cardiac conduction. Encompasses interactions such as signaling or attachment between one cell and another cell, between a cell and an extracellular matrix, or between a cell and any other aspect of its environment. Also known as: SA node cardiac muscle cell to atrial cardiac muscle cell communication, SA node cardiomyocyte to atrial cardiomyocyte communication, SAN cardiomyocyte to atrial cardiomyocyte communication, sinoatrial node cardiomyocyte to atrial cardiomyocyte communication, sinus node cardiomyocyte to atrial cardiomyocyte communication